{
  "term_label": "mitogen-activated protein kinase kinase binding",
  "term_id": "GO:0031434",
  "gene": "UniProtKB:Q92519",
  "gene_symbol": "TRIB2",
  "gene_name": "Tribbles homolog 2"
}